{
  "gene_name": "Leucine-rich repeat neuronal protein 2",
  "gene_symbol": "LRRN2",
  "term_label": "signaling receptor activity",
  "term_id": "GO:0038023",
  "gene": "UniProtKB:O75325"
}